{
  "gene": "UniProtKB:P55064",
  "gene_symbol": "AQP5",
  "term_id": "GO:0015670",
  "gene_name": "Aquaporin-5",
  "term_label": "carbon dioxide transport"
}